{
  "gene_symbol": "ATG14",
  "gene_name": "Beclin 1-associated autophagy-related key regulator",
  "gene": "UniProtKB:Q6ZNE5",
  "term_label": "mitophagy",
  "term_id": "GO:0000423"
}